myosin II light chain binding [GO:0032033] (molecular function) Definition: Binding to a light chain of a myosin II complex. Relationships: is a type of GO:0032027; is a type of myosin II binding [GO:0045159] Sources: GOC:mah